{
  "gene": "UniProtKB:Q15165",
  "term_label": "response to toxic substance",
  "term_id": "GO:0009636",
  "gene_symbol": "PON2",
  "gene_name": "Serum paraoxonase_arylesterase 2"
}